{
  "gene_symbol": "DNAJC12",
  "gene": "UniProtKB:Q9UKB3",
  "term_label": "Unknown molecular function",
  "term_id": "UNKNOWN:0001",
  "gene_name": "DnaJ homolog subfamily C member 12"
}